{
  "gene_symbol": "EDNRB",
  "term_label": "endothelin receptor activity",
  "gene": "UniProtKB:P24530",
  "term_id": "GO:0004962",
  "gene_name": "Endothelin receptor type B"
}